regulation of ornithine catabolic process [GO:1903266] (biological process) References: PMID:12679340 Sources: GOC:TermGenie, GOC:bhm, GO_REF:0000058 Subtypes: negative regulation of ornithine catabolic process [GO:1903267], positive regulation of ornithine catabolic process [GO:1903268] Also known as: regulation of ornithine breakdown, regulation of ornithine catabolism, regulation of ornithine degradation Definition: Any process that modulates the frequency, rate or extent of ornithine catabolic process. Relationships: is a type of regulation of catabolic process [GO:0009894]; is a type of regulation of ornithine metabolic process [GO:0090368]; regulates L-ornithine catabolic process [GO:0006593] Note: An example of this is ARGI in Saccharomyces cerevisiae (P00812) in PMID:12679340 (inferred from direct assay).